{
  "term_id": "UNKNOWN:0003",
  "gene": "UniProtKB:Q5VVP1",
  "gene_name": "Spermatogenesis-associated protein 31A6",
  "gene_symbol": "SPATA31A6",
  "term_label": "Unknown cellular component"
}